chloroplast large ribosomal subunit [GO:0022628] (cellular component) Relationships: is a type of plastid large ribosomal subunit [GO:0000311]; BFO_0000050 chloroplast ribosome [GO:0043253] Definition: The large subunit of a ribosome contained within a chloroplast. Sources: GOC:mtg_sensu Also known as: chloroplast ribosomal LSU complex, chloroplast ribosomal large subunit complex